{
  "gene_name": "Mitotic-spindle organizing protein 1",
  "term_id": "GO:0051415",
  "term_label": "microtubule nucleation by interphase microtubule organizing center",
  "gene": "UniProtKB:Q08AG7",
  "gene_symbol": "MZT1"
}